{
  "gene_symbol": "GP6",
  "term_id": "GO:0038063",
  "gene": "UniProtKB:Q9HCN6",
  "gene_name": "Platelet glycoprotein VI",
  "term_label": "collagen-activated tyrosine kinase receptor signaling pathway"
}